regulation of cardiolipin metabolic process [GO:1900208] (biological process) Definition: Any process that modulates the frequency, rate or extent of cardiolipin metabolic process. Relationships: is a type of regulation of phospholipid metabolic process [GO:1903725]; regulates cardiolipin metabolic process [GO:0032048] Also known as: regulation of cardiolipin metabolism, regulation of diphosphatidylglycerol metabolic process, regulation of diphosphatidylglycerol metabolism Subtypes: negative regulation of cardiolipin metabolic process [GO:1900209], positive regulation of cardiolipin metabolic process [GO:1900210] Sources: GOC:TermGenie